semaphorin-plexin signaling pathway involved in neuron projection guidance [GO:1902285] (biological process) Definition: Any semaphorin-plexin signaling pathway that is involved in neuron projection guidance. References: PMID:22790009 Sources: GOC:BHF, GOC:TermGenie, GOC:rl Also known as: semaphorin-plexin signaling pathway involved in neuron process guidance, semaphorin-plexin signaling pathway involved in neuron protrusion guidance, semaphorin-plexin signaling pathway involved in neuronal cell projection guidance, semaphorin-plexin signalling pathway involved in neuron process guidance, semaphorin-plexin signalling pathway involved in neuron projection guidance, semaphorin-plexin signalling pathway involved in neuron protrusion guidance, semaphorin-plexin signalling pathway involved in neuronal cell projection guidance, semaphorin-plexin signaling pathway involved in neurite guidance, semaphorin-plexin signalling pathway involved in neurite guidance Relationships: is a type of GO:0071526; is part of GO:0097485 Subtypes: semaphorin-plexin signaling pathway involved in dendrite guidance [GO:1902286], GO:1902287